{
  "gene": "UniProtKB:P19875",
  "term_label": "Unknown biological process",
  "gene_name": "C-X-C motif chemokine 2",
  "gene_symbol": "CXCL2",
  "term_id": "UNKNOWN:0002"
}